{
  "gene_symbol": "CDKN1B",
  "term_id": "GO:0045930",
  "gene_name": "Cyclin-dependent kinase inhibitor 1B",
  "term_label": "negative regulation of mitotic cell cycle",
  "gene": "UniProtKB:P46527"
}